{
  "gene_symbol": "SLC1A4",
  "gene_name": "Neutral amino acid transporter A",
  "term_id": "GO:0015180",
  "term_label": "L-alanine transmembrane transporter activity",
  "gene": "UniProtKB:P43007"
}